{
  "term_id": "UNKNOWN:0001",
  "gene_symbol": "CFAP210",
  "gene": "UniProtKB:Q0VFZ6",
  "term_label": "Unknown molecular function",
  "gene_name": "Cilia- and flagella- associated protein 210"
}